{
  "term_label": "Unknown cellular component",
  "gene_symbol": "TAB1",
  "gene_name": "TGF-beta-activated kinase 1 and MAP3K7-binding protein 1",
  "term_id": "UNKNOWN:0003",
  "gene": "UniProtKB:Q15750"
}